spine synapse [GO:0106033] (cellular component) Also known as: dendritic spine synapse Definition: A type of synapse occurring between an axon and a dendritic spine. Relationships: is a type of asymmetric synapse [GO:0032279] References: PMID:15028757